{
  "gene_symbol": "LRRC74A",
  "term_label": "Unknown cellular component",
  "gene_name": "Leucine-rich repeat-containing protein 74A",
  "gene": "UniProtKB:Q0VAA2",
  "term_id": "UNKNOWN:0003"
}